{
  "gene_symbol": "PLAU",
  "term_id": "GO:0033628",
  "gene_name": "Urokinase-type plasminogen activator",
  "gene": "UniProtKB:P00749",
  "term_label": "regulation of cell adhesion mediated by integrin"
}